reciprocal homologous recombination [GO:0140527] (biological process) References: PMID:17846636 Relationships: is a type of homologous recombination [GO:0035825] Subtypes: reciprocal meiotic recombination [GO:0007131] Definition: A DNA recombination process that results in the bidirectional exchange of genetic material between highly homologous DNA molecules.